{
  "gene_symbol": "KCNQ2",
  "term_id": "GO:0071805",
  "gene": "UniProtKB:O43526",
  "gene_name": "Potassium voltage-gated channel subfamily KQT member 2",
  "term_label": "potassium ion transmembrane transport"
}